detection of redox state [GO:0051776] (biological process) Definition: The series of events in which a chemical stimulus indicating redox state is received and converted into a molecular signal. Redox state refers to the balance of oxidized versus reduced forms of electron donors and acceptors in an organelle, cell or organ; plastoquinone, glutathione (GSH/GSSG), and nicotinamide nucleotides (NAD+/NADH and NADP+/NADPH) are among the most important. Relationships: is a type of GO:0009593; is a type of GO:0051775 Also known as: redox sensing References: PMID:15131240, PMID:16987039 Sources: GOC:mah